{
  "gene": "UniProtKB:Q9Y2F5",
  "gene_name": "Little elongation complex subunit 1",
  "term_id": "GO:0008023",
  "gene_symbol": "ICE1",
  "term_label": "transcription elongation factor complex"
}